{
  "gene_symbol": "DUSP29",
  "term_label": "cytoplasm",
  "term_id": "GO:0005737",
  "gene_name": "Dual specificity phosphatase 29",
  "gene": "UniProtKB:Q68J44"
}